{
  "gene_name": "Transport and Golgi organization protein 1 homolog",
  "gene_symbol": "MIA3",
  "term_id": "GO:0005789",
  "gene": "UniProtKB:Q5JRA6",
  "term_label": "endoplasmic reticulum membrane"
}